{
  "term_label": "nucleus",
  "gene_name": "NEDD4-binding protein 2-like 2",
  "term_id": "GO:0005634",
  "gene": "UniProtKB:Q92802",
  "gene_symbol": "N4BP2L2"
}